{
  "gene_name": "Structural maintenance of chromosomes protein 4",
  "term_label": "nucleus",
  "gene_symbol": "SMC4",
  "term_id": "GO:0005634",
  "gene": "UniProtKB:Q9NTJ3"
}